type III interferon production [GO:0034343] (biological process) Subtypes: interleukin-28A production [GO:0072627], interleukin-28B production [GO:0072629], interleukin-29 production [GO:0072631] Relationships: is a type of cytokine production [GO:0001816] Regulation: regulated by regulation of type III interferon production [GO:0034344]; negatively regulated by GO:0034345; positively regulated by GO:0034346 Definition: The appearance of type III interferon due to biosynthesis or secretion following a cellular stimulus, resulting in an increase in its intracellular or extracellular levels. Interferon lambda is the only member of the type III interferon found so far. References: PMID:15546383, PMID:16734557 Sources: GOC:add, ISBN:0126896631 Note: Note that IL-28A, IL-28B, and IL-29 are types of interferon-lambda. This term is in the subset of terms that should not be used for direct gene product annotation. Instead, select one of the 'regulation' children terms. Also known as: type III IFN production, type III interferon secretion